{
  "gene_symbol": "MPC2",
  "term_id": "GO:0006850",
  "gene": "UniProtKB:O95563",
  "term_label": "pyruvate import into mitochondria",
  "gene_name": "Mitochondrial pyruvate carrier 2"
}